morphogenesis of an epithelial fold [GO:0060571] (BP) Sources: GOC:dph Relationships: is a type of morphogenesis of an epithelium [GO:0002009] Subtypes: GO:0001842, morphogenesis of an epithelial fold involved in embryonic heart tube formation [GO:0003152], myocardial epithelial involution involved in heart jogging [GO:0003304], GO:0007374, neural fold bending [GO:0021503], neural fold folding [GO:0021505], invagination involved in gastrulation with mouth forming second [GO:0055109], involution involved in gastrulation with mouth forming second [GO:0055110], morphogenesis of an epithelial bud [GO:0060572], pouch outgrowth involved in semicircular canal formation [GO:0060878] Definition: The morphogenetic process in which an epithelial sheet bends along a linear axis. Also known as: epithelial folding, folding of an epithelial sheet